{
  "term_label": "maintenance of synapse structure",
  "term_id": "GO:0099558",
  "gene_name": "Cerebellin-4",
  "gene_symbol": "CBLN4",
  "gene": "UniProtKB:Q9NTU7"
}